{
  "term_label": "macrophage activation",
  "gene_symbol": "IL13",
  "gene_name": "Interleukin-13",
  "term_id": "GO:0042116",
  "gene": "UniProtKB:P35225"
}